{
  "term_label": "Unknown cellular component",
  "term_id": "UNKNOWN:0003",
  "gene_name": "Acid phosphatase type 7",
  "gene_symbol": "ACP7",
  "gene": "UniProtKB:Q6ZNF0"
}